fungiform papilla development [GO:0061196] (biological process) Sources: GOC:dph Relationships: is a type of anatomical structure development [GO:0048856]; is part of GO:0043586 Definition: The progression of the fungiform papilla over time, from its formation to the mature structure. The fungiform papilla is a mushroom-shaped papilla of the tongue.